H2A-H2B histone complex chaperone activity [GO:0000511] (molecular function) Relationships: is a type of histone chaperone activity [GO:0140713] Definition: A histone chaperone that carries a H2A-H2B histone complex. References: PMID:28053344 Also known as: H2A-H2B histone carrier activity